{
  "term_label": "RNA polymerase II cis-regulatory region sequence-specific DNA binding",
  "gene_name": "Krueppel-like factor 16",
  "gene_symbol": "KLF16",
  "term_id": "GO:0000978",
  "gene": "UniProtKB:Q9BXK1"
}